positive regulation of post-transcriptional gene silencing by RNA [GO:1900370] (biological process) Definition: Any process that activates or increases the frequency, rate or extent of post-transcriptional gene silencing by RNA. References: PMID:22412382 Sources: GOC:TermGenie, GOC:kmv Also known as: activation of RNAi, positive regulation of PTGS, positive regulation of RNA interference, positive regulation of RNAi, up regulation of RNA interference, up regulation of RNAi, up-regulation of RNA interference, up-regulation of RNAi, upregulation of RNA interference, upregulation of RNAi, activation of RNA interference Relationships: is a type of positive regulation of post-transcriptional gene silencing [GO:0060148]; is a type of regulation of post-transcriptional gene silencing by regulatory ncRNA [GO:1900368]; positively regulates regulatory ncRNA-mediated post-transcriptional gene silencing [GO:0035194] Subtypes: positive regulation of miRNA-mediated gene silencing [GO:2000637]